{
  "term_label": "trace-amine receptor activity",
  "gene_name": "Trace amine-associated receptor 1",
  "gene_symbol": "TAAR1",
  "gene": "UniProtKB:Q96RJ0",
  "term_id": "GO:0001594"
}